negative regulation of protein autophosphorylation [GO:0031953] (biological process) Sources: GOC:mah Also known as: down regulation of protein amino acid autophosphorylation, down-regulation of protein amino acid autophosphorylation, downregulation of protein amino acid autophosphorylation, negative regulation of protein amino acid autophosphorylation, inhibition of protein amino acid autophosphorylation Definition: Any process that stops, prevents or decreases the rate of the phosphorylation by a protein of one or more of its own residues. Relationships: is a type of negative regulation of protein phosphorylation [GO:0001933]; is a type of GO:0031952; has part negative regulation of protein kinase activity [GO:0006469]; negatively regulates protein autophosphorylation [GO:0046777] Subtypes: negative regulation of peptidyl-tyrosine autophosphorylation [GO:1900085]